chromatin loop anchoring activity [GO:0140587] (molecular function) Relationships: is a type of GO:0031490; is a type of DNA-DNA tethering activity [GO:0106260] Also known as: DNA loop binding, chromosomal loop binding References: PMID:32213323 Subtypes: promoter-enhancer loop anchoring activity [GO:0140585], promoter-terminator loop anchoring activity [GO:0140586] Definition: Bridging together two DNA loop anchors together, maintaining a chromatin loop.